{
  "term_label": "cytoplasm",
  "gene": "UniProtKB:P31327",
  "gene_symbol": "CPS1",
  "term_id": "GO:0005737",
  "gene_name": "Carbamoyl-phosphate synthase [ammonia], mitochondrial"
}